heart rudiment formation [GO:0003315] (biological process) Relationships: is a type of anatomical structure formation involved in morphogenesis [GO:0048646]; is part of heart rudiment morphogenesis [GO:0003314] Sources: GOC:mtg_heart Definition: The developmental process pertaining to the initial formation of the heart rudiment. Also known as: heart cone formation